{
  "term_id": "GO:0003723",
  "gene_name": "Heterogeneous nuclear ribonucleoprotein A_B",
  "term_label": "RNA binding",
  "gene": "UniProtKB:Q99729",
  "gene_symbol": "HNRNPAB"
}